{
  "gene": "UniProtKB:Q96JI7",
  "gene_symbol": "SPG11",
  "term_label": "axonogenesis",
  "gene_name": "Spatacsin",
  "term_id": "GO:0007409"
}